{
  "gene_name": "Pro-FMRFamide-related neuropeptide FF",
  "gene_symbol": "NPFF",
  "term_id": "GO:0001664",
  "gene": "UniProtKB:O15130",
  "term_label": "G protein-coupled receptor binding"
}